{
  "gene_symbol": "MBD3L3",
  "term_id": "GO:0000122",
  "gene": "UniProtKB:A6NE82",
  "gene_name": "Putative methyl-CpG-binding domain protein 3-like 3",
  "term_label": "negative regulation of transcription by RNA polymerase II"
}